cysteine-type deNEDDylase activity [GO:0140757] (molecular function) Definition: An thiol-dependent isopeptidase activity that cleaves NEDD8 from a target protein to which it is conjugated. References: PMID:25628956 Relationships: is a type of cysteine-type peptidase activity [GO:0008234]; is a type of deNEDDylase activity [GO:0019784]